negative regulation of dendritic cell chemotaxis [GO:2000509] (biological process) Relationships: is a type of negative regulation of leukocyte chemotaxis [GO:0002689]; is a type of GO:0071676; is a type of GO:2000508; negatively regulates GO:0002407 Sources: GOC:obol Subtypes: negative regulation of myeloid dendritic cell chemotaxis [GO:2000528] Definition: Any process that stops, prevents or reduces the frequency, rate or extent of dendritic cell chemotaxis.